{
  "gene": "UniProtKB:O75818",
  "term_label": "ribonuclease MRP activity",
  "term_id": "GO:0000171",
  "gene_name": "Ribonuclease P protein subunit p40",
  "gene_symbol": "RPP40"
}